miltiradiene catabolic process [GO:1901945] (biological process) Definition: The chemical reactions and pathways resulting in the breakdown of miltiradiene. Also known as: miltiradiene breakdown, miltiradiene catabolism, miltiradiene degradation References: PMID:22027823 Sources: GOC:TermGenie Relationships: is_a terpene catabolic process [GO:0046247]